larval visceral muscle development [GO:0007523] (BP) Sources: GOC:jid Relationships: is a type of visceral muscle development [GO:0007522]; BFO_0000050 larval development [GO:0002164] Definition: The process whose specific outcome is the progression of the larval visceral muscle over time, from its formation to the mature structure.